response to mechanical stimulus [GO:0009612] (biological process) Sources: GOC:hb Definition: Any process that results in a change in state or activity of a cell or an organism (in terms of movement, secretion, enzyme production, gene expression, etc.) as a result of a mechanical stimulus. Also known as: mechanical stimulus response, chemi-mechanical coupling Subtypes: GO:0009652, GO:0010996, response to muscle stretch [GO:0035994], detection of mechanical stimulus [GO:0050982], cellular response to mechanical stimulus [GO:0071260], response to ultrasound [GO:1990478] Relationships: is a type of GO:0009605; is a type of GO:0009628